{
  "term_id": "GO:0000149",
  "gene": "UniProtKB:Q9BSW7",
  "gene_name": "Synaptotagmin-17",
  "term_label": "SNARE binding",
  "gene_symbol": "SYT17"
}